{
  "term_id": "GO:0031463",
  "gene_name": "Calicin",
  "term_label": "Cul3-RING ubiquitin ligase complex",
  "gene_symbol": "CCIN",
  "gene": "UniProtKB:Q13939"
}